{
  "gene": "UniProtKB:A6NFN3",
  "term_label": "nucleus",
  "gene_symbol": "RBFOX3",
  "gene_name": "RNA binding protein fox-1 homolog 3",
  "term_id": "GO:0005634"
}